{
  "gene_name": "NADPH oxidase 3",
  "term_id": "GO:0016175",
  "term_label": "superoxide-generating NAD(P)H oxidase activity",
  "gene_symbol": "NOX3",
  "gene": "UniProtKB:Q9HBY0"
}